chicken-wire-like collagen network [GO:0140154] (cellular component) Definition: Network-forming collagens can either form a chicken-wire-like network or a hexagonal network. Collagen type IV forms a chicken-wire-like structure and is found in the basement membrane. Relationships: is a type of collagen network [GO:0098645]; is part of collagenous component of basement membrane [GO:0140143] References: PMID:21421911, PMID:21421915, PMID:31387942